{
  "gene_name": "Protein-serine O-palmitoleoyltransferase porcupine",
  "gene": "UniProtKB:Q9H237",
  "term_label": "lipid modification",
  "term_id": "GO:0030258",
  "gene_symbol": "PORCN"
}